{
  "gene_name": "A disintegrin and metalloproteinase with thrombospondin motifs 18",
  "gene_symbol": "ADAMTS18",
  "gene": "UniProtKB:Q8TE60",
  "term_label": "metalloendopeptidase activity",
  "term_id": "GO:0004222"
}